{
  "gene": "UniProtKB:Q9H9F9",
  "gene_symbol": "ACTR5",
  "term_id": "GO:0031011",
  "gene_name": "Actin-related protein 5",
  "term_label": "Ino80 complex"
}